response to peptidoglycan [GO:0032494] (biological process) Sources: GOC:add, ISBN:0721601464 Subtypes: detection of peptidoglycan [GO:0032499], cellular response to peptidoglycan [GO:0071224] Definition: Any process that results in a change in state or activity of an organism (in terms of movement, secretion, enzyme production, gene expression, etc.) as a result of a peptidoglycan stimulus. Peptidoglycan is a bacterial cell wall macromolecule. Relationships: is a type of response to molecule of bacterial origin [GO:0002237]; is a type of GO:1901698; is a type of response to oxygen-containing compound [GO:1901700]